{
  "term_id": "GO:0005544",
  "term_label": "calcium-dependent phospholipid binding",
  "gene_name": "Copine-4",
  "gene": "UniProtKB:Q96A23",
  "gene_symbol": "CPNE4"
}